{
  "term_label": "mitochondrion",
  "term_id": "GO:0005739",
  "gene_symbol": "COX10",
  "gene": "UniProtKB:Q12887",
  "gene_name": "Protoheme IX farnesyltransferase, mitochondrial"
}